{
  "term_label": "Unknown molecular function",
  "term_id": "UNKNOWN:0001",
  "gene_name": "Zinc finger protein 830",
  "gene_symbol": "ZNF830",
  "gene": "UniProtKB:Q96NB3"
}